attachment of mitotic spindle microtubules to kinetochore [GO:0051315] (biological process) Subtypes: GO:0099607, mitotic sister chromatid biorientation [GO:1990758] Also known as: attachment of spindle microtubules to kinetochore involved in mitosis, attachment of spindle microtubules to kinetochore involved in mitotic sister chromatid segregation, attachment of spindle microtubules to mitotic chromosome, attachment of spindle microtubules to kinetochore during mitosis, mitotic bipolar attachment References: PMID:26258632, PMID:26705896 Sources: GOC:ai, GOC:clt, GOC:dph, GOC:tb Regulation: regulated by GO:1902423; negatively regulated by negative regulation of attachment of mitotic spindle microtubules to kinetochore [GO:1902424]; positively regulated by positive regulation of attachment of mitotic spindle microtubules to kinetochore [GO:1902425] Definition: The cellular process in which spindle microtubules become physically associated with the proteins making up the kinetochore complex in mitosis. Note: This class covers transient, lateral attachment to microtubules as well as stable, correctly oriented, end-on attachment (biorientation) Relationships: is a type of GO:0008608; is a type of GO:1903047; is part of mitotic metaphase chromosome alignment [GO:0007080]